olfactory cortex development [GO:0021989] (biological process) Definition: The progression of the olfactory cortex over time from its initial formation until its mature state. The olfactory cortex is involved in the perception of smell. It receives input from the olfactory bulb and is responsible for the identification of odors. Sources: GOC:cls, GOC:dgh, GOC:dph, GOC:jid, GO_REF:0000021 Relationships: is a type of GO:0048856; is part of olfactory lobe development [GO:0021988]